{
  "gene": "UniProtKB:Q9H4A4",
  "gene_symbol": "RNPEP",
  "gene_name": "Aminopeptidase B",
  "term_id": "GO:0006508",
  "term_label": "proteolysis"
}